{
  "term_label": "DNA-binding transcription factor activity, RNA polymerase II-specific",
  "term_id": "GO:0000981",
  "gene_symbol": "HOMEZ",
  "gene_name": "Homeobox and leucine zipper protein Homez",
  "gene": "UniProtKB:Q8IX15"
}